{
  "gene": "UniProtKB:P51813",
  "gene_symbol": "BMX",
  "term_label": "non-membrane spanning protein tyrosine kinase activity",
  "gene_name": "Cytoplasmic tyrosine-protein kinase BMX",
  "term_id": "GO:0004715"
}